{
  "term_id": "GO:0000977",
  "gene_symbol": "LHX8",
  "gene": "UniProtKB:Q68G74",
  "gene_name": "LIM_homeobox protein Lhx8",
  "term_label": "RNA polymerase II transcription regulatory region sequence-specific DNA binding"
}